{
  "term_label": "sodium ion transmembrane transport",
  "gene": "UniProtKB:Q16515",
  "term_id": "GO:0035725",
  "gene_symbol": "ASIC2",
  "gene_name": "Acid-sensing ion channel 2"
}